{
  "gene": "UniProtKB:A6NM36",
  "term_label": "Unknown molecular function",
  "gene_name": "Leucine-rich repeat-containing protein 30",
  "term_id": "UNKNOWN:0001",
  "gene_symbol": "LRRC30"
}